{
  "term_label": "Unknown cellular component",
  "term_id": "UNKNOWN:0003",
  "gene_symbol": "NAA38",
  "gene": "UniProtKB:Q9BRA0",
  "gene_name": "N-alpha-acetyltransferase 38, NatC auxiliary subunit"
}